{
  "term_label": "DNA replication initiation",
  "gene": "UniProtKB:Q8WTT2",
  "gene_symbol": "NOC3L",
  "term_id": "GO:0006270",
  "gene_name": "Nucleolar complex protein 3 homolog"
}